very-long-chain 3-oxoacyl-CoA reductase activity [GO:0141040] (molecular function) References: PMID:16564093, PMID:19763486 Sources: RHEA:48680 Relationships: is a type of GO:0016616 Definition: Catalysis of the reaction: a very-long-chain (3R)-3-hydroxyacyl-CoA + NADP+ = a very-long-chain 3-oxoacyl-CoA + H+ + NADPH. This reaction is the second (reduction) step of the four-step fatty acid elongation cycle in the endoplasmic reticulum that extends fatty acids of C-16 or longer with an additional 2-C unit.